sn-glycerol 1-phosphatase activity [GO:0000121] (molecular function) Definition: Catalysis of the reaction: H2O + sn-glycerol 1-phosphate = glycerol + phosphate. Also known as: glycerol-1-phosphatase activity, alpha-glycerol phosphatase activity, alpha-glycerophosphatase activity, glycerol 3-phosphatase activity, glycerol 3-phosphate phosphohydrolase activity, glycerol-1-phosphate phosphohydrolase activity, glycerol-3-phosphate phosphatase activity Sources: RHEA:46084 Relationships: is a type of phosphatase activity [GO:0016791]